{
  "term_id": "GO:0003918",
  "gene_name": "DNA topoisomerase 2-alpha",
  "term_label": "DNA topoisomerase type II (double strand cut, ATP-hydrolyzing) activity",
  "gene_symbol": "TOP2A",
  "gene": "UniProtKB:P11388"
}